{
  "gene_name": "Probable E3 ubiquitin-protein ligase TRIML2",
  "term_label": "cytoplasm",
  "term_id": "GO:0005737",
  "gene": "UniProtKB:Q8N7C3",
  "gene_symbol": "TRIML2"
}